{
  "gene": "UniProtKB:Q8N823",
  "gene_symbol": "ZNF611",
  "term_id": "GO:0006357",
  "term_label": "regulation of transcription by RNA polymerase II",
  "gene_name": "Zinc finger protein 611"
}